{
  "gene": "UniProtKB:O00425",
  "gene_symbol": "IGF2BP3",
  "term_label": "mRNA 3'-UTR binding",
  "gene_name": "Insulin-like growth factor 2 mRNA-binding protein 3",
  "term_id": "GO:0003730"
}